{
  "gene_name": "RNA-binding protein 33",
  "term_label": "Unknown biological process",
  "term_id": "UNKNOWN:0002",
  "gene_symbol": "RBM33",
  "gene": "UniProtKB:Q96EV2"
}